{
  "gene_symbol": "TMEM278",
  "gene_name": "Transmembrane protein 88B",
  "term_label": "plasma membrane",
  "term_id": "GO:0005886",
  "gene": "UniProtKB:A6NKF7"
}